{
  "term_id": "GO:0005634",
  "gene": "UniProtKB:O60518",
  "gene_symbol": "RANBP6",
  "gene_name": "Ran-binding protein 6",
  "term_label": "nucleus"
}